ear morphogenesis [GO:0042471] (BP) Relationships: is a type of embryonic organ morphogenesis [GO:0048562]; is a type of sensory organ morphogenesis [GO:0090596]; is part of ear development [GO:0043583] Also known as: hearing organ morphogenesis Sources: GOC:jl, ISBN:0192801023 Definition: The process in which the anatomical structures of the ear are generated and organized. The ear is the sense organ in vertebrates that is specialized for the detection of sound, and the maintenance of balance. Includes the outer ear and middle ear, which collect and transmit sound waves; and the inner ear, which contains the organs of balance and (except in fish) hearing. Also includes the pinna, the visible part of the outer ear, present in some mammals.